{
  "term_label": "glutamate-cysteine ligase activity",
  "gene_name": "Glutamate--cysteine ligase catalytic subunit",
  "term_id": "GO:0004357",
  "gene_symbol": "GCLC",
  "gene": "UniProtKB:P48506"
}